{
  "gene_name": "Lanosterol synthase",
  "gene_symbol": "LSS",
  "term_id": "GO:0005811",
  "gene": "UniProtKB:P48449",
  "term_label": "lipid droplet"
}